{
  "gene_symbol": "CDKN1C",
  "gene": "UniProtKB:P49918",
  "term_id": "UNKNOWN:0001",
  "term_label": "Unknown molecular function",
  "gene_name": "Cyclin-dependent kinase inhibitor 1C"
}